{
  "term_label": "transcription cis-regulatory region binding",
  "term_id": "GO:0000976",
  "gene": "UniProtKB:Q6P1X5",
  "gene_symbol": "TAF2",
  "gene_name": "Transcription initiation factor TFIID subunit 2"
}